{
  "term_id": "GO:0055056",
  "gene_name": "Solute carrier family 2, facilitated glucose transporter member 14",
  "term_label": "D-glucose transmembrane transporter activity",
  "gene": "UniProtKB:Q8TDB8",
  "gene_symbol": "SLC2A14"
}